{
  "gene_name": "Visinin-like protein 1",
  "term_label": "regulation of signal transduction",
  "gene": "UniProtKB:P62760",
  "term_id": "GO:0009966",
  "gene_symbol": "VSNL1"
}